sulfate adenylyltransferase activity [GO:0004779] (molecular function) Sources: GOC:mah Definition: Catalysis of the transfer of an adenylyl group from an adenosine nucleotide (ATP or ADP) to sulfate, forming adenylylsulfate. Relationships: is a type of adenylyltransferase activity [GO:0070566] Also known as: sulphate adenylyltransferase activity Subtypes: GO:0004780, sulfate adenylyltransferase (ATP) activity [GO:0004781]